{
  "term_label": "endosome organization",
  "gene_name": "Pleckstrin homology domain-containing family F member 1",
  "gene_symbol": "PLEKHF1",
  "gene": "UniProtKB:Q96S99",
  "term_id": "GO:0007032"
}